{
  "gene": "UniProtKB:Q6PJG2",
  "term_id": "GO:0000118",
  "term_label": "histone deacetylase complex",
  "gene_symbol": "MIDEAS",
  "gene_name": "Mitotic deacetylase-associated SANT domain protein"
}